spinal cord anterior/posterior patterning [GO:0021512] (BP) Definition: The process that regulates the coordinated growth and differentiation that establishes the non-random anterior-posterior spatial arrangement of the spinal cord. Sources: GOC:cls, GOC:dgh, GOC:dph, GOC:jid, GO_REF:0000021 Also known as: spinal cord anterior-posterior patterning, spinal cord rostrocaudal patterning Relationships: is a type of anterior/posterior pattern specification [GO:0009952]; is part of spinal cord patterning [GO:0021511]